{
  "gene_symbol": "RPS6KA3",
  "gene_name": "Ribosomal protein S6 kinase alpha-3",
  "term_id": "GO:0005654",
  "term_label": "nucleoplasm",
  "gene": "UniProtKB:P51812"
}